{
  "gene_symbol": "METTL5",
  "term_label": "rRNA methylation",
  "gene": "UniProtKB:Q9NRN9",
  "gene_name": "rRNA N6-adenosine-methyltransferase METTL5",
  "term_id": "GO:0031167"
}